{
  "term_label": "odorant binding",
  "gene": "UniProtKB:Q96RC9",
  "term_id": "GO:0005549",
  "gene_name": "Olfactory receptor 8B4",
  "gene_symbol": "OR8B4"
}